{
  "gene": "UniProtKB:Q9Y4A9",
  "term_label": "olfactory receptor activity",
  "gene_symbol": "OR10H1",
  "gene_name": "Olfactory receptor 10H1",
  "term_id": "GO:0004984"
}